vanillin biosynthetic process [GO:0042189] (biological process) Relationships: is a type of vanillin metabolic process [GO:0018982]; is a type of aldehyde biosynthetic process [GO:0046184]; is_a GO:0046189; is a type of ether biosynthetic process [GO:1901503] Definition: The chemical reactions and pathways resulting in the formation of vanillin, an aromatic hydrocarbon which occurs naturally in black vanilla bean pods. Sources: GOC:jl Also known as: vanillic aldehyde biosynthesis, vanillic aldehyde biosynthetic process, vanillin anabolism, vanillin biosynthesis, vanillin formation, vanillin synthesis